leukotriene D4 catabolic process [GO:1901749] (biological process) Relationships: is a type of leukotriene catabolic process [GO:0036100]; is_a GO:0043603; is a type of sulfur compound catabolic process [GO:0044273]; is a type of icosanoid catabolic process [GO:1901523] Definition: The chemical reactions and pathways resulting in the breakdown of leukotriene D4. Sources: GOC:TermGenie, GOC:yaf Also known as: leukotriene D4 breakdown, leukotriene D4 catabolism, leukotriene D4 degradation